{
  "gene_symbol": "FOXD1",
  "term_id": "UNKNOWN:0003",
  "gene": "UniProtKB:Q16676",
  "term_label": "Unknown cellular component",
  "gene_name": "Forkhead box protein D1"
}